{
  "gene": "UniProtKB:Q9Y467",
  "term_id": "GO:0000981",
  "gene_name": "Sal-like protein 2",
  "term_label": "DNA-binding transcription factor activity, RNA polymerase II-specific",
  "gene_symbol": "SALL2"
}